{
  "term_id": "GO:0000976",
  "term_label": "transcription cis-regulatory region binding",
  "gene": "UniProtKB:Q8N4W9",
  "gene_name": "Zinc finger protein 808",
  "gene_symbol": "ZNF808"
}